{
  "gene_symbol": "PCDHA7",
  "gene_name": "Protocadherin alpha-7",
  "term_label": "plasma membrane",
  "term_id": "GO:0005886",
  "gene": "UniProtKB:Q9UN72"
}